{
  "term_label": "microtubule cytoskeleton organization",
  "gene_name": "Tubulin--tyrosine ligase",
  "gene": "UniProtKB:Q8NG68",
  "term_id": "GO:0000226",
  "gene_symbol": "TTL"
}